{
  "term_label": "90S preribosome",
  "term_id": "GO:0030686",
  "gene_symbol": "UTP20",
  "gene_name": "Small subunit processome component 20 homolog",
  "gene": "UniProtKB:O75691"
}